{
  "term_id": "GO:0070971",
  "gene_symbol": "SEC16B",
  "gene_name": "Protein transport protein Sec16B",
  "term_label": "endoplasmic reticulum exit site",
  "gene": "UniProtKB:Q96JE7"
}